{
  "gene_name": "Fibroblast growth factor 10",
  "gene_symbol": "FGF10",
  "term_id": "GO:0042056",
  "gene": "UniProtKB:O15520",
  "term_label": "chemoattractant activity"
}